{
  "term_label": "Unknown cellular component",
  "gene_name": "Uncharacterized protein",
  "term_id": "UNKNOWN:0003",
  "gene": "UniProtKB:A0A3B3IRQ3",
  "gene_symbol": "LOC112267897"
}